mu-type opioid receptor binding [GO:0031852] (molecular function) Definition: Binding to a mu-type opioid receptor. Sources: GOC:mah, GOC:nln, GOC:sl Also known as: mu-type opioid receptor ligand, morphine receptor binding Relationships: is a type of opioid receptor binding [GO:0031628]